regulation of gamma-aminobutyric acid catabolic process [GO:1901715] (biological process) Relationships: is a type of regulation of amino acid metabolic process [GO:0006521]; is a type of regulation of catabolic process [GO:0009894]; is a type of GO:0062012; regulates gamma-aminobutyric acid catabolic process [GO:0009450] Subtypes: negative regulation of gamma-aminobutyric acid catabolic process [GO:1901716], positive regulation of gamma-aminobutyric acid catabolic process [GO:1901717] Definition: Any process that modulates the frequency, rate or extent of gamma-aminobutyric acid catabolic process. Sources: GOC:TermGenie Also known as: regulation of 4-aminobutanoate catabolic process, regulation of 4-aminobutanoate catabolism, regulation of 4-aminobutyrate catabolic process, regulation of 4-aminobutyrate catabolism, regulation of GABA catabolic process, regulation of GABA catabolism, regulation of gamma-aminobutyric acid breakdown, regulation of gamma-aminobutyric acid catabolism, regulation of gamma-aminobutyric acid degradation